{
  "gene": "UniProtKB:Q8TF72",
  "gene_symbol": "SHROOM3",
  "term_id": "GO:0051015",
  "gene_name": "Protein Shroom3",
  "term_label": "actin filament binding"
}